positive regulation of cardiac ventricle development [GO:1904414] (biological process) References: PMID:19590510 Sources: GOC:TermGenie, GO_REF:0000058 Definition: Any process that activates or increases the frequency, rate or extent of cardiac ventricle development. Relationships: is a type of positive regulation of developmental process [GO:0051094]; is a type of positive regulation of multicellular organismal process [GO:0051240]; is a type of GO:1904412; positively regulates cardiac ventricle development [GO:0003231] Also known as: up regulation of cardiac ventricle development, up-regulation of cardiac ventricle development, upregulation of cardiac ventricle development, activation of cardiac ventricle development